{
  "term_label": "Unknown molecular function",
  "gene": "UniProtKB:A0A804HJT0",
  "gene_name": "Uncharacterized protein",
  "term_id": "UNKNOWN:0001",
  "gene_symbol": "A0A804HJT0"
}